positive regulation of metula development [GO:0070804] (biological process) Definition: Any process that activates or increases the frequency, rate or extent of metula development, a process that leads to the formation of metulae. Metulae are elongated mononucleate cells that bud from the surface of the conidiophore tip. Sources: GOC:mah Relationships: is a type of positive regulation of cell development [GO:0010720]; is a type of GO:0070802; is a type of positive regulation of reproductive process [GO:2000243]; positively regulates metula development [GO:0070789]